{
  "term_label": "nucleus",
  "gene_symbol": "CDCA4",
  "gene": "UniProtKB:Q9BXL8",
  "gene_name": "Cell division cycle-associated protein 4",
  "term_id": "GO:0005634"
}